{
  "gene": "UniProtKB:P09884",
  "gene_name": "DNA polymerase alpha catalytic subunit",
  "term_label": "DNA-directed DNA polymerase activity",
  "term_id": "GO:0003887",
  "gene_symbol": "POLA1"
}